{
  "gene_symbol": "DEF6",
  "gene": "UniProtKB:Q9H4E7",
  "gene_name": "Differentially expressed in FDCP 6 homolog",
  "term_id": "UNKNOWN:0002",
  "term_label": "Unknown biological process"
}